{
  "term_id": "GO:0000028",
  "gene": "UniProtKB:P39019",
  "gene_name": "Small ribosomal subunit protein eS19",
  "term_label": "ribosomal small subunit assembly",
  "gene_symbol": "RPS19"
}